{
  "gene_name": "Nucleoside diphosphate-linked moiety X motif 17",
  "gene": "UniProtKB:P0C025",
  "term_id": "GO:0006742",
  "term_label": "NADP+ catabolic process",
  "gene_symbol": "NUDT17"
}